{
  "gene_symbol": "RELL2",
  "term_label": "positive regulation of cell-substrate adhesion",
  "gene": "UniProtKB:Q8NC24",
  "term_id": "GO:0010811",
  "gene_name": "RELT-like protein 2"
}